{
  "term_id": "GO:0033209",
  "gene_name": "COMM domain-containing protein 7",
  "gene_symbol": "COMMD7",
  "term_label": "tumor necrosis factor-mediated signaling pathway",
  "gene": "UniProtKB:Q86VX2"
}